{
  "term_id": "GO:0032590",
  "gene_symbol": "GABRG3",
  "gene_name": "Gamma-aminobutyric acid receptor subunit gamma-3",
  "term_label": "dendrite membrane",
  "gene": "UniProtKB:Q99928"
}